{
  "gene_name": "Protein TANC1",
  "term_id": "UNKNOWN:0001",
  "term_label": "Unknown molecular function",
  "gene_symbol": "TANC1",
  "gene": "UniProtKB:Q9C0D5"
}